Golgi membrane priming complex assembly [GO:0048195] (biological process) Definition: The aggregation, arrangement and bonding together of a set of components to form a membrane priming complex. An incoming coat component recognizes both GTPase and a membrane protein to form the priming complex. References: PMID:10219233 Sources: GOC:jid, ISBN:0716731363 Also known as: formation of Golgi membrane priming complex, formation of dictyosome membrane priming complex Relationships: is a type of protein-containing complex assembly [GO:0065003]; is part of Golgi transport vesicle coating [GO:0048200]